{
  "term_id": "GO:0015035",
  "gene": "UniProtKB:Q8N4Q1",
  "gene_name": "Mitochondrial intermembrane space import and assembly protein 40",
  "gene_symbol": "CHCHD4",
  "term_label": "protein-disulfide reductase activity"
}